negative regulation of foraging behavior [GO:1903369] (biological process) References: PMID:8677262 Sources: GOC:TermGenie, GOC:mr, GO_REF:0000058 Also known as: down regulation of foraging behavior, down-regulation of foraging behavior, downregulation of foraging behavior, inhibition of foraging behavior Relationships: is a type of negative regulation of behavior [GO:0048521]; is_a GO:1903368; negatively regulates GO:0060756 Definition: Any process that stops, prevents or reduces the frequency, rate or extent of foraging behavior.